Kit signaling pathway [GO:0038109] (biological process) Relationships: is_a cell surface receptor protein tyrosine kinase signaling pathway [GO:0007169]; is a type of cytokine-mediated signaling pathway [GO:0019221]; is part of cellular response to stem cell factor stimulus [GO:0036216] References: PMID:16129412 Sources: GOC:nhn, GOC:signaling Also known as: Kit signalling pathway, SCF signaling pathway, stem cell factor receptor signaling pathway, stem cell factor signaling pathway Definition: The series of molecular signals initiated by the binding of stem cell factor to the tyrosine kinase receptor KIT on the surface of a target cell, and ending with regulation of a downstream cellular process, e.g. transcription. Stem cell factor (KIT ligand) binding to the receptor Kit mediates receptor dimerization, activation of its intrinsic tyrosine kinase activity and autophosphorylation. The activated receptor then phosphorylates various substrates, thereby activating distinct signaling cascades within the cell that trigger a change in state or activity of the cell. Regulation: regulated by regulation of Kit signaling pathway [GO:1900234]; negatively regulated by negative regulation of Kit signaling pathway [GO:1900235]; positively regulated by positive regulation of Kit signaling pathway [GO:1900236]